glycine reductase activity [GO:0030699] (molecular function) Relationships: is a type of oxidoreductase activity, acting on X-H and Y-H to form an X-Y bond, with a disulfide as acceptor [GO:0050485] Also known as: acetyl-phosphate ammonia:thioredoxin disulfide oxidoreductase (glycine-forming) Definition: Catalysis of the reaction: acetyl phosphate + H2O + NH4 + thioredoxin disulfide = glycine + H+ + phosphate + thioredoxin. Sources: EC:1.21.4.2, RHEA:12232